{
  "gene": "UniProtKB:Q9N2K0",
  "term_id": "UNKNOWN:0003",
  "gene_symbol": "Q9N2K0",
  "gene_name": "HERV-H_2q24.3 provirus ancestral Env polyprotein",
  "term_label": "Unknown cellular component"
}